endoplasmic reticulum lumen [GO:0005788] (cellular component) Also known as: ER cisterna, ER lumen, cisternal lumen, endoplasmic reticulum cisterna Sources: ISBN:0198547684 Subtypes: sarcoplasmic reticulum lumen [GO:0033018], GO:0048237, smooth endoplasmic reticulum lumen [GO:0048238], perinuclear endoplasmic reticulum lumen [GO:0099020], cortical endoplasmic reticulum lumen [GO:0099021] Definition: The volume enclosed by the membranes of the endoplasmic reticulum. Relationships: is a type of intracellular organelle lumen [GO:0070013]; is part of GO:0005783